regulation of protein-containing complex assembly [GO:0043254] (biological process) Definition: Any process that modulates the frequency, rate or extent of protein complex assembly. Sources: GOC:jl Also known as: regulation of protein complex assembly Relationships: is a type of regulation of cellular component biogenesis [GO:0044087]; is a type of regulation of cellular component organization [GO:0051128]; regulates GO:0065003 Subtypes: GO:0001928, regulation of COPII vesicle coating [GO:0003400], regulation of synaptic vesicle priming [GO:0010807], GO:0031333, GO:0031334, GO:0032271, regulation of protein oligomerization [GO:0032459], regulation of integrin activation [GO:0033623], regulation of SNARE complex assembly [GO:0035542], GO:0043520, regulation of RNA polymerase II transcription preinitiation complex assembly [GO:0045898], regulation of pseudohyphal septin ring assembly [GO:0062164], regulation of podosome assembly [GO:0071801], GO:0090034, regulation of high-density lipoprotein particle assembly [GO:0090107], regulation of kinetochore assembly [GO:0090234], regulation of proteasome assembly [GO:0090364], regulation of AIM2 inflammasome complex assembly [GO:0140971], regulation of nodal receptor complex assembly [GO:1900123], GO:1900225, regulation of starch utilization system complex assembly [GO:1900512], regulation of formation of translation initiation ternary complex [GO:1901190], GO:1901193, GO:1902442, regulation of assembly of large subunit precursor of preribosome [GO:1902627], regulation of death-inducing signaling complex assembly [GO:1903072], GO:1903872, regulation of VCP-NPL4-UFD1 AAA ATPase complex assembly [GO:1904239], regulation of Wnt-Frizzled-LRP5/6 complex assembly [GO:1904711], regulation of shelterin complex assembly [GO:1904790], regulation of beta-catenin-TCF complex assembly [GO:1904863], regulation of telomerase catalytic core complex assembly [GO:1904882], regulation of apoptosome assembly [GO:1905100], regulation of clathrin coat assembly [GO:1905443], regulation of eukaryotic translation initiation factor 4F complex assembly [GO:1905535], regulation of FACT complex assembly [GO:1905644], GO:1905864, regulation of mediator complex assembly [GO:2001176]